{
  "gene": "UniProtKB:Q5SZJ8",
  "term_id": "GO:0045746",
  "gene_symbol": "BEND6",
  "gene_name": "BEN domain-containing protein 6",
  "term_label": "negative regulation of Notch signaling pathway"
}